{
  "gene": "UniProtKB:Q96NB1",
  "term_id": "GO:0036064",
  "gene_name": "Centrosomal protein 20",
  "term_label": "ciliary basal body",
  "gene_symbol": "CEP20"
}